negative regulation of monocyte activation [GO:0150102] (biological process) Definition: Any process that stops, prevents or reduces the frequency, rate or extent of monocyte activation. Relationships: is_a GO:0002695; negatively regulates monocyte activation [GO:0042117] Also known as: repression of monocyte activation References: PMID:15597323 Sources: GOC:aruk